{
  "term_label": "intermediate filament organization",
  "gene_symbol": "KRT80",
  "term_id": "GO:0045109",
  "gene": "UniProtKB:Q6KB66",
  "gene_name": "Keratin, type II cytoskeletal 80"
}